{
  "gene": "UniProtKB:Q8N140",
  "term_label": "Smc5-Smc6 complex",
  "gene_symbol": "EID3",
  "gene_name": "EP300-interacting inhibitor of differentiation 3",
  "term_id": "GO:0030915"
}